{
  "gene_symbol": "H1-2",
  "term_label": "double-stranded DNA binding",
  "gene": "UniProtKB:P16403",
  "gene_name": "Histone H1.2",
  "term_id": "GO:0003690"
}